{
  "gene_symbol": "BSN",
  "gene_name": "Protein bassoon",
  "gene": "UniProtKB:Q9UPA5",
  "term_label": "presynaptic active zone assembly",
  "term_id": "GO:1904071"
}